positive regulation of biosynthetic process [GO:0009891] (biological process) Also known as: positive regulation of anabolism, positive regulation of biosynthesis, positive regulation of formation, positive regulation of synthesis, up regulation of biosynthetic process, up-regulation of biosynthetic process, upregulation of biosynthetic process, activation of biosynthetic process, stimulation of biosynthetic process Relationships: is_a regulation of biosynthetic process [GO:0009889]; is_a positive regulation of metabolic process [GO:0009893]; positively regulates GO:0009058 Sources: GOC:go_curators Subtypes: positive regulation of flavonoid biosynthetic process [GO:0009963], positive regulation of macromolecule biosynthetic process [GO:0010557], positive regulation of nucleotide biosynthetic process [GO:0030810], positive regulation of collagen biosynthetic process [GO:0032967], positive regulation of nitric oxide biosynthetic process [GO:0045429], positive regulation of gluconeogenesis [GO:0045722], GO:0046886, positive regulation of lipid biosynthetic process [GO:0046889], GO:0050747, positive regulation of taurine biosynthetic process [GO:0062090], GO:0062162, positive regulation of (R)-mevalonic acid biosynthetic process [GO:0106109], positive regulation of UDP-N-acetylglucosamine biosynthetic process [GO:0106280], GO:0140176, positive regulation of raffinose biosynthetic process [GO:1900093], GO:1900185, positive regulation of methanofuran biosynthetic process [GO:1900353], positive regulation of secondary metabolite biosynthetic process [GO:1900378], positive regulation of austinol biosynthetic process [GO:1900642], positive regulation of naphtho-gamma-pyrone biosynthetic process [GO:1900848], GO:1900851, positive regulation of hexadecanal biosynthetic process [GO:1900904], positive regulation of olefin biosynthetic process [GO:1900913], positive regulation of methanophenazine biosynthetic process [GO:1900964], positive regulation of sarcinapterin biosynthetic process [GO:1900973], positive regulation of tatiopterin biosynthetic process [GO:1900976], positive regulation of phenazine biosynthetic process [GO:1900982], positive regulation of spermidine biosynthetic process [GO:1901307], positive regulation of tetrapyrrole biosynthetic process [GO:1901465], positive regulation of alkane biosynthetic process [GO:1901579], positive regulation of fumagillin biosynthetic process [GO:1902092], positive regulation of alcohol biosynthetic process [GO:1902932], positive regulation of dopamine biosynthetic process [GO:1903181], GO:1903428, positive regulation of lactose biosynthetic process [GO:1903536], positive regulation of glutathione biosynthetic process [GO:1903788], positive regulation of pyrimidine-containing compound salvage [GO:1903931], positive regulation of ubiquinone biosynthetic process [GO:1904775], positive regulation of hydrogen sulfide biosynthetic process [GO:1904828], positive regulation of vitamin E biosynthetic process [GO:1904966], positive regulation of quinolinate biosynthetic process [GO:1904986], positive regulation of serotonin biosynthetic process [GO:1905629], positive regulation of trypanothione biosynthetic process [GO:1905724], positive regulation of acetylcholine biosynthetic process [GO:1905923], GO:2000284 Definition: Any process that activates or increases the frequency, rate or extent of the chemical reactions and pathways resulting in the formation of substances.